{
  "gene_name": "E3 ubiquitin-protein ligase SMURF1",
  "term_id": "GO:0043161",
  "term_label": "proteasome-mediated ubiquitin-dependent protein catabolic process",
  "gene": "UniProtKB:Q9HCE7",
  "gene_symbol": "SMURF1"
}